deoxynucleoside phosphate kinase activity, GTP as phosphate donor [GO:0106369] (MF) Relationships: is a type of phosphotransferase activity, phosphate group as acceptor [GO:0016776]; is_a nucleobase-containing compound kinase activity [GO:0019205] References: PMID:20497505 Sources: RHEA:62124 Definition: Catalysis of the reaction: a 2'-deoxyribonucleoside 5'-phosphate + GTP = a 2'-deoxyribonucleoside 5'-diphosphate + GDP.